{
  "gene_symbol": "STRN4",
  "term_id": "GO:0030425",
  "gene": "UniProtKB:Q9NRL3",
  "gene_name": "Striatin-4",
  "term_label": "dendrite"
}